bromide peroxidase activity [GO:0019806] (molecular function) Definition: Catalysis of the reaction: 2 R-H + 2 bromide + H2O2 = 2 R-Br + 2 H2O. Enzymes with this activity often accept other halide ions as substrates, including chloride and iodide. Sources: EC:1.11.1.18 Also known as: bromoperoxidase activity Relationships: is a type of haloperoxidase activity [GO:0140905]